{
  "gene_symbol": "ADRA1A",
  "term_label": "alpha1-adrenergic receptor activity",
  "gene_name": "Alpha-1A adrenergic receptor",
  "gene": "UniProtKB:P35348",
  "term_id": "GO:0004937"
}